{
  "term_id": "GO:0032998",
  "gene_symbol": "FCER1G",
  "term_label": "Fc-epsilon receptor I complex",
  "gene_name": "High affinity immunoglobulin epsilon receptor subunit gamma",
  "gene": "UniProtKB:P30273"
}